programmed DNA elimination by chromosome breakage [GO:0031052] (biological process) Relationships: is a type of programmed DNA elimination [GO:0031049] Definition: Regulated cleavage of the developing macronuclear genome at a limited number of chromosome breakage sites (CBS). The macronuclear destined segment (MDS) sequence adjacent to the CBS (or separated from it by a BES) receives a macronuclear telomere following chromosome breakage. Also known as: chromosome breakage References: PMID:15956677, PMID:25303953, PMID:32165395 Sources: GOC:ns Note: Note that this term refers to breakage of chromosomes during normal DNA well characterized in ciliates but also present in many vertebrates; it is not to be used for DNA damage or other abnormal occurrences.